cellular response to non-ionic osmotic stress [GO:0071471] (biological process) Relationships: is a type of response to non-ionic osmotic stress [GO:0010335]; is_a cellular response to osmotic stress [GO:0071470] Definition: Any process that results in a change in state or activity of a cell (in terms of movement, secretion, enzyme production, gene expression, etc.) as a result of a stimulus indicating an increase or decrease in the concentration of non-ionic solutes (e.g. mannitol, sorbitol) in the environment. Sources: GOC:mah